{
  "gene_name": "Unconventional myosin-Ia",
  "term_label": "cytoplasm",
  "term_id": "GO:0005737",
  "gene_symbol": "MYO1A",
  "gene": "UniProtKB:Q9UBC5"
}